{
  "gene_symbol": "RPA4",
  "term_label": "DNA replication factor A complex",
  "term_id": "GO:0005662",
  "gene_name": "Replication protein A 30 kDa subunit",
  "gene": "UniProtKB:Q13156"
}